{
  "gene_symbol": "ANAPC7",
  "gene_name": "Anaphase-promoting complex subunit 7",
  "term_label": "positive regulation of mitotic metaphase/anaphase transition",
  "term_id": "GO:0045842",
  "gene": "UniProtKB:Q9UJX3"
}